response to asparaginase [GO:0061480] (biological process) Relationships: is a type of response to chemical [GO:0042221] Sources: GOC:dph Definition: Any process that results in a change in state or activity of a cell or an organism (in terms of movement, secretion, enzyme production, gene expression, etc.) as a result of an asparaginase stimulus.